{
  "gene_symbol": "KIF22",
  "gene_name": "Kinesin-like protein KIF22",
  "term_id": "GO:0003777",
  "gene": "UniProtKB:Q14807",
  "term_label": "microtubule motor activity"
}